{
  "gene": "UniProtKB:Q9BTV6",
  "term_label": "cytoplasm",
  "gene_symbol": "DPH7",
  "gene_name": "Diphthine methyltransferase",
  "term_id": "GO:0005737"
}